perineuronal net [GO:0072534] (cellular component) References: PMID:18364019 Sources: GOC:sl Definition: A dense extracellular matrix (ECM) that forms around many neuronal cell bodies and dendrites late in development and is responsible for synaptic stabilization in the adult brain. Also known as: PNN Relationships: is a type of perisynaptic extracellular matrix [GO:0098966]